{
  "gene": "UniProtKB:Q5JXX7",
  "term_id": "UNKNOWN:0003",
  "gene_name": "Transmembrane protein 31",
  "gene_symbol": "TMEM31",
  "term_label": "Unknown cellular component"
}